{
  "term_label": "podocyte differentiation",
  "term_id": "GO:0072112",
  "gene_name": "Receptor-type tyrosine-protein phosphatase O",
  "gene_symbol": "PTPRO",
  "gene": "UniProtKB:Q16827"
}